{
  "gene_name": "Putative uncharacterized protein ADARB2-AS1",
  "term_id": "UNKNOWN:0003",
  "term_label": "Unknown cellular component",
  "gene_symbol": "ADARB2-AS1",
  "gene": "UniProtKB:A8MUL3"
}